{
  "term_id": "GO:0046512",
  "gene_name": "Neutral ceramidase",
  "gene": "UniProtKB:Q9NR71",
  "term_label": "sphingosine biosynthetic process",
  "gene_symbol": "ASAH2"
}